{
  "term_id": "GO:0005829",
  "gene_name": "Casein kinase II subunit alpha'",
  "gene": "UniProtKB:P19784",
  "term_label": "cytosol",
  "gene_symbol": "CSNK2A2"
}